{
  "gene_symbol": "DYNC2LI1",
  "term_id": "GO:0005868",
  "gene_name": "Cytoplasmic dynein 2 light intermediate chain 1",
  "gene": "UniProtKB:Q8TCX1",
  "term_label": "cytoplasmic dynein complex"
}